{
  "gene_symbol": "COX4I2",
  "term_id": "UNKNOWN:0001",
  "gene_name": "Cytochrome c oxidase subunit 4 isoform 2, mitochondrial",
  "gene": "UniProtKB:Q96KJ9",
  "term_label": "Unknown molecular function"
}